{
  "gene_symbol": "FBXW8",
  "term_label": "ciliary basal body",
  "gene_name": "F-box_WD repeat-containing protein 8",
  "gene": "UniProtKB:Q8N3Y1",
  "term_id": "GO:0036064"
}